{
  "gene_symbol": "AADAT",
  "gene": "UniProtKB:Q8N5Z0",
  "term_id": "GO:0016212",
  "gene_name": "Kynurenine_alpha-aminoadipate aminotransferase, mitochondrial",
  "term_label": "kynurenine-oxoglutarate transaminase activity"
}